{
  "gene_symbol": "NDUFA3",
  "gene_name": "NADH dehydrogenase [ubiquinone] 1 alpha subcomplex subunit 3",
  "term_label": "respiratory chain complex I",
  "gene": "UniProtKB:O95167",
  "term_id": "GO:0045271"
}